{
  "term_label": "Unknown molecular function",
  "gene": "UniProtKB:Q6ZUI0",
  "term_id": "UNKNOWN:0001",
  "gene_name": "Tumor protein p63-regulated gene 1 protein",
  "gene_symbol": "TPRG1"
}